{
  "term_id": "GO:0008104",
  "gene_name": "Septin-1",
  "gene_symbol": "SEPTIN1",
  "gene": "UniProtKB:Q8WYJ6",
  "term_label": "intracellular protein localization"
}